{
  "term_label": "dUTP catabolic process",
  "gene_name": "Deoxyuridine 5'-triphosphate nucleotidohydrolase, mitochondrial",
  "gene_symbol": "DUT",
  "gene": "UniProtKB:P33316",
  "term_id": "GO:0046081"
}